{
  "gene": "UniProtKB:Q9Y2U2",
  "gene_symbol": "KCNK7",
  "gene_name": "Potassium channel subfamily K member 7",
  "term_label": "potassium ion transmembrane transport",
  "term_id": "GO:0071805"
}